{
  "gene": "UniProtKB:Q01970",
  "term_id": "GO:0005516",
  "gene_symbol": "PLCB3",
  "gene_name": "1-phosphatidylinositol 4,5-bisphosphate phosphodiesterase beta-3",
  "term_label": "calmodulin binding"
}